{
  "gene": "UniProtKB:O95258",
  "term_id": "GO:0005743",
  "gene_name": "Brain mitochondrial carrier protein 1",
  "gene_symbol": "SLC25A14",
  "term_label": "mitochondrial inner membrane"
}